{
  "term_id": "GO:0005737",
  "term_label": "cytoplasm",
  "gene_name": "Homer protein homolog 1",
  "gene": "UniProtKB:Q86YM7",
  "gene_symbol": "HOMER1"
}